zymogen granule exocytosis [GO:0070625] (biological process) References: PMID:17442889 Sources: GOC:BHF, GOC:vk Definition: The release of intracellular molecules contained within the zymogen granule by fusion of the granule with the plasma membrane of the oocyte, requiring calcium ions. Relationships: is a type of calcium-ion regulated exocytosis [GO:0017156]